negative regulation of R8 cell spacing in compound eye [GO:0045469] (biological process) References: PMID:11880339 Sources: GOC:dph, GOC:tb Relationships: is a type of regulation of R8 cell spacing in compound eye [GO:0045468] Also known as: down regulation of R8 spacing, down-regulation of R8 spacing, downregulation of R8 spacing, inhibition of R8 spacing Definition: Any process that stops or prevents the correct R8 cell spacing pattern in a compound eye.